{
  "term_label": "RNA polymerase II cis-regulatory region sequence-specific DNA binding",
  "gene": "UniProtKB:O94916",
  "gene_symbol": "NFAT5",
  "term_id": "GO:0000978",
  "gene_name": "Nuclear factor of activated T-cells 5"
}